organic anion transport [GO:0015711] (biological process) Definition: The directed movement of organic anions into, out of or within a cell, or between cells, by means of some agent such as a transporter or pore. Organic anions are atoms or small molecules with a negative charge which contain carbon in covalent linkage. Sources: GOC:ai, GOC:krc Relationships: is a type of transport [GO:0006810] Subtypes: glycerophosphodiester transmembrane transport [GO:0001407], ferric-enterobactin import into cell [GO:0015685], bicarbonate transport [GO:0015701], GO:0015747, glucose-6-phosphate transport [GO:0015760], CMP-N-acetylneuraminate transmembrane transport [GO:0015782], UDP-glucose transmembrane transport [GO:0015786], UDP-N-acetylgalactosamine transmembrane transport [GO:0015789], UDP-xylose transmembrane transport [GO:0015790], GO:0015794, ADP transport [GO:0015866], ATP transport [GO:0015867], coenzyme A transport [GO:0015880], FAD transport [GO:0015883], tetracycline transmembrane transport [GO:0015904], GO:0015916, thiamine pyrophosphate transmembrane transport [GO:0030974], GO:0031921, riboflavin transport [GO:0032218], myo-inositol hexakisphosphate transport [GO:0033272], GO:0034635, triose phosphate transmembrane transport [GO:0035436], alkanesulfonate transmembrane transport [GO:0042918], enterobactin transport [GO:0042930], sodium-dependent organic anion transport [GO:0043251], sodium-independent organic anion transport [GO:0043252], carboxylic acid transport [GO:0046942], 3'-phosphoadenosine 5'-phosphosulfate transport [GO:0046963], GO:0070730, cGMP transport [GO:0070731], glycerol-2-phosphate transmembrane transport [GO:0070811], GO:0070837, phytochelatin transport [GO:0071993], UDP-galactose transmembrane transport [GO:0072334], AMP transport [GO:0080121], cyclic-GMP-AMP transmembrane import across plasma membrane [GO:0140361], UDP-beta-L-arabinofuranose import into Golgi lumen [GO:0140821], isopentenyl pyrophosphate import into mitochondrion [GO:0170046], GO:1902389, GO:1902558, UDP-N-acetylglucosamine transmembrane transport [GO:1990569]